{
  "gene_name": "Inactive rhomboid protein 2",
  "gene": "UniProtKB:Q6PJF5",
  "term_id": "GO:0005789",
  "gene_symbol": "RHBDF2",
  "term_label": "endoplasmic reticulum membrane"
}